{
  "term_label": "negative regulation of RIG-I signaling pathway",
  "gene": "UniProtKB:Q96C10",
  "gene_symbol": "DHX58",
  "gene_name": "ATP-dependent RNA helicase DHX58",
  "term_id": "GO:0039536"
}